{
  "gene": "UniProtKB:P61968",
  "gene_name": "LIM domain transcription factor LMO4",
  "term_id": "GO:0021520",
  "term_label": "spinal cord motor neuron cell fate specification",
  "gene_symbol": "LMO4"
}